{
  "gene_name": "Beta-1,3-galactosyl-O-glycosyl-glycoprotein beta-1,6-N-acetylglucosaminyltransferase 7",
  "term_id": "UNKNOWN:0002",
  "term_label": "Unknown biological process",
  "gene": "UniProtKB:Q6ZNI0",
  "gene_symbol": "GCNT7"
}